{
  "term_id": "GO:0005634",
  "term_label": "nucleus",
  "gene": "UniProtKB:P01100",
  "gene_name": "Protein c-Fos",
  "gene_symbol": "FOS"
}